{
  "gene_name": "Neurotensin receptor type 1",
  "term_id": "GO:0005886",
  "term_label": "plasma membrane",
  "gene": "UniProtKB:P30989",
  "gene_symbol": "NTSR1"
}